{
  "term_label": "nucleoplasm",
  "gene_symbol": "EID2B",
  "gene_name": "EP300-interacting inhibitor of differentiation 2B",
  "gene": "UniProtKB:Q96D98",
  "term_id": "GO:0005654"
}